{
  "term_id": "UNKNOWN:0003",
  "gene_symbol": "Q6ZRM9",
  "term_label": "Unknown cellular component",
  "gene": "UniProtKB:Q6ZRM9",
  "gene_name": "Putative uncharacterized protein FLJ46235"
}